{
  "gene_name": "Conserved oligomeric Golgi complex subunit 5",
  "gene": "UniProtKB:Q9UP83",
  "gene_symbol": "COG5",
  "term_id": "GO:0017119",
  "term_label": "Golgi transport complex"
}